{
  "gene_symbol": "TUBB2B",
  "gene": "UniProtKB:Q9BVA1",
  "term_id": "GO:0000226",
  "term_label": "microtubule cytoskeleton organization",
  "gene_name": "Tubulin beta-2B chain"
}